{
  "term_id": "UNKNOWN:0002",
  "gene_name": "Cystatin-D",
  "term_label": "Unknown biological process",
  "gene_symbol": "CST5",
  "gene": "UniProtKB:P28325"
}